germ plasm [GO:0060293] (cellular component) Sources: GOC:dph Definition: Differentiated cytoplasm associated with a pole of an oocyte, egg or early embryo that will be inherited by the cells that will give rise to the germ line. Relationships: is a type of pole plasm [GO:0045495]